{
  "gene_name": "Protein FAM90A27P",
  "gene_symbol": "FAM90A27P",
  "gene": "UniProtKB:A6NNH2",
  "term_id": "UNKNOWN:0002",
  "term_label": "Unknown biological process"
}